{
  "gene_name": "Tubulin-specific chaperone D",
  "term_id": "GO:0034333",
  "term_label": "adherens junction assembly",
  "gene": "UniProtKB:Q9BTW9",
  "gene_symbol": "TBCD"
}